{
  "gene_symbol": "SNED1",
  "gene": "UniProtKB:Q8TER0",
  "term_label": "Unknown cellular component",
  "gene_name": "Sushi, nidogen and EGF-like domain-containing protein 1",
  "term_id": "UNKNOWN:0003"
}